NAD+ biosynthetic process [GO:0009435] (biological process) Definition: The chemical reactions and pathways resulting in the formation of nicotinamide adenine dinucleotide (NAD+), a coenzyme that interconverts with its reduced form, NADH, in many redox and catabolic reactions. NAD+ is derived from various sources including vitamin B3. Also known as: NAD (oxidized) biosynthesis, NAD (oxidized) biosynthetic process, NAD (reduced) biosynthesis, NAD (reduced) biosynthetic process, NAD anabolism, NAD biosynthesis, NAD biosynthetic process, NAD formation, NAD synthesis, NADH biosynthesis, NADH biosynthetic process, nicotinamide adenine dinucleotide biosynthesis, nicotinamide adenine dinucleotide biosynthetic process, oxidized NAD biosynthesis, oxidized NAD biosynthetic process, oxidized nicotinamide adenine dinucleotide biosynthesis, oxidized nicotinamide adenine dinucleotide biosynthetic process, reduced NAD biosynthesis, reduced NAD biosynthetic process, reduced nicotinamide adenine dinucleotide biosynthesis, reduced nicotinamide adenine dinucleotide biosynthetic process Relationships: is a type of purine nucleotide biosynthetic process [GO:0006164]; is a type of nicotinamide nucleotide biosynthetic process [GO:0019359]; is a type of NAD+ metabolic process [GO:0019674] Subtypes: 'de novo' NAD+ biosynthetic process from L-tryptophan [GO:0034354], NAD+ biosynthetic process via the salvage pathway [GO:0034355], 'de novo' NAD+ biosynthetic process from L-aspartate [GO:0034628] References: PMID:28648096